negative regulation of autophagosome maturation [GO:1901097] (biological process) Relationships: is_a GO:0016242; is a type of negative regulation of protein-containing complex disassembly [GO:0043242]; is a type of regulation of autophagosome maturation [GO:1901096]; RO_0002212 autophagosome maturation [GO:0097352] Definition: Any process that stops, prevents or reduces the frequency, rate or extent of autophagosome maturation. Also known as: down regulation of autophagic vacuole fusion, down regulation of autophagic vacuole maturation, down regulation of autophagosome maturation, down-regulation of autophagic vacuole fusion, down-regulation of autophagic vacuole maturation, down-regulation of autophagosome maturation, downregulation of autophagic vacuole fusion, downregulation of autophagic vacuole maturation, downregulation of autophagosome maturation, inhibition of autophagosome maturation, negative regulation of autophagic vacuole fusion, negative regulation of autophagosome fusion, down regulation of amphisome-lysosome fusion, down regulation of autolysosome formation, down regulation of fusion of autophagosome with lysosome, down-regulation of amphisome-lysosome fusion, down-regulation of autolysosome formation, down-regulation of fusion of autophagosome with lysosome, downregulation of amphisome-lysosome fusion, downregulation of autolysosome formation, downregulation of fusion of autophagosome with lysosome, inhibition of amphisome-lysosome fusion, inhibition of autolysosome formation, inhibition of autophagic vacuole fusion, inhibition of autophagic vacuole maturation, inhibition of fusion of autophagosome with lysosome, negative regulation of amphisome-lysosome fusion, negative regulation of autolysosome formation, negative regulation of fusion of autophagosome with lysosome References: PMID:10436019, PMID:21383079 Sources: GOC:TermGenie, GOC:autophagy